thigmotaxis [GO:0001966] (biological process) Sources: GOC:dph Relationships: is a type of behavior [GO:0007610] Definition: The directed movement of an animal in response to touch. Also known as: taxis in response to mechanical stimulus, stereotaxis, taxis in response to touch stimulus